{
  "term_id": "UNKNOWN:0002",
  "gene_symbol": "SPATA9",
  "gene_name": "Spermatogenesis-associated protein 9",
  "term_label": "Unknown biological process",
  "gene": "UniProtKB:Q9BWV2"
}